regulation of mechanosensory behavior [GO:1905790] (biological process) References: PMID:8692859 Sources: GOC:TermGenie, GO_REF:0000058 Relationships: is a type of GO:0032101; is a type of regulation of behavior [GO:0050795]; regulates mechanosensory behavior [GO:0007638] Subtypes: GO:1905791, GO:1905792 Definition: Any process that modulates the frequency, rate or extent of mechanosensory behavior. Also known as: regulation of behavioral response to mechanical stimulus, regulation of behavioural response to mechanical stimulus, regulation of mechanosensory behaviour